{
  "gene": "UniProtKB:Q7Z7K2",
  "term_id": "GO:0005634",
  "term_label": "nucleus",
  "gene_name": "Zinc finger protein 467",
  "gene_symbol": "ZNF467"
}